{
  "gene_name": "Spindle and kinetochore-associated protein 2",
  "gene": "UniProtKB:Q8WVK7",
  "term_label": "outer kinetochore",
  "gene_symbol": "SKA2",
  "term_id": "GO:0000940"
}